{
  "gene": "UniProtKB:Q14117",
  "gene_name": "Dihydropyrimidinase",
  "term_id": "GO:0006208",
  "term_label": "pyrimidine nucleobase catabolic process",
  "gene_symbol": "DPYS"
}